{
  "gene_name": "SH3 and cysteine-rich domain-containing protein",
  "term_label": "Unknown cellular component",
  "term_id": "UNKNOWN:0003",
  "gene": "UniProtKB:Q99469",
  "gene_symbol": "STAC"
}